{
  "term_id": "UNKNOWN:0003",
  "gene_symbol": "KIAA1671",
  "gene": "UniProtKB:Q9BY89",
  "term_label": "Unknown cellular component",
  "gene_name": "Uncharacterized protein KIAA1671"
}